{
  "gene": "UniProtKB:O43613",
  "gene_symbol": "HCRTR1",
  "term_id": "GO:0005886",
  "gene_name": "Orexin_Hypocretin receptor type 1",
  "term_label": "plasma membrane"
}